{
  "term_id": "UNKNOWN:0001",
  "gene_symbol": "FAM90A11P",
  "gene": "UniProtKB:A0A8V8TNH8",
  "gene_name": "Family with sequence similarity 90 member A11, pseudogene",
  "term_label": "Unknown molecular function"
}